{
  "gene_symbol": "RAC1",
  "term_label": "motor neuron axon guidance",
  "gene": "UniProtKB:P63000",
  "term_id": "GO:0008045",
  "gene_name": "Ras-related C3 botulinum toxin substrate 1"
}